{
  "gene_symbol": "BSPRY",
  "term_id": "GO:0061630",
  "gene": "UniProtKB:Q5W0U4",
  "term_label": "ubiquitin protein ligase activity",
  "gene_name": "B box and SPRY domain-containing protein"
}